swim bladder formation [GO:0048797] (biological process) Also known as: gas bladder biosynthesis, gas bladder formation Relationships: is_a GO:0048645; is part of swim bladder morphogenesis [GO:0048795] Sources: GOC:mh Definition: The process that gives rise to the swim bladder. This process pertains to the initial formation of a structure from unspecified parts. The swim bladder is used by some fishes to maintain buoyancy and may function in addition as a sound producing organ, a sound receptor, and a respiratory organ.